dTDP-rhamnose biosynthetic process [GO:0019305] (biological process) Also known as: dTDP-rhamnose anabolism, dTDP-rhamnose biosynthesis, dTDP-rhamnose formation, dTDP-rhamnose synthesis Sources: GOC:ai Relationships: is a type of GO:0009226 Definition: The chemical reactions and pathways resulting in the formation of dTDP-rhamnose, a substance composed of rhamnose in glycosidic linkage with deoxyribosylthymine diphosphate.